{
  "gene_name": "DENN domain-containing protein 1B",
  "gene_symbol": "DENND1B",
  "gene": "UniProtKB:Q6P3S1",
  "term_id": "GO:0032456",
  "term_label": "endocytic recycling"
}